notochord cell vacuolation [GO:0060036] (biological process) Definition: The assembly and arrangement of a vacuole within a cell of the notochord. References: PMID:10964477 Sources: GOC:cb, GOC:dph Relationships: is a type of vacuole organization [GO:0007033]; is part of notochord cell development [GO:0060035]